{
  "gene": "UniProtKB:P32519",
  "gene_name": "ETS-related transcription factor Elf-1",
  "term_label": "DNA-binding transcription factor activity, RNA polymerase II-specific",
  "term_id": "GO:0000981",
  "gene_symbol": "ELF1"
}